{
  "gene_symbol": "CDK19",
  "term_id": "GO:0005829",
  "gene_name": "Cyclin-dependent kinase 19",
  "term_label": "cytosol",
  "gene": "UniProtKB:Q9BWU1"
}